{
  "gene": "UniProtKB:Q6UXS9",
  "gene_name": "Inactive caspase-12",
  "gene_symbol": "CASP12",
  "term_id": "GO:0005829",
  "term_label": "cytosol"
}